{
  "term_id": "GO:0005737",
  "gene_name": "Serine_threonine-protein kinase 33",
  "gene": "UniProtKB:Q9BYT3",
  "term_label": "cytoplasm",
  "gene_symbol": "STK33"
}